{
  "gene": "UniProtKB:O60684",
  "gene_symbol": "KPNA6",
  "term_id": "GO:0008139",
  "gene_name": "Importin subunit alpha-7",
  "term_label": "nuclear localization sequence binding"
}